negative regulation of 17-methylnonadec-1-ene biosynthetic process [GO:1900957] (biological process) Sources: GOC:TermGenie, GOC:mengo_curators Definition: Any process that stops, prevents or reduces the frequency, rate or extent of 17-methylnonadec-1-ene biosynthetic process. Relationships: is a type of negative regulation of olefin biosynthetic process [GO:1900912]; is a type of GO:1900956; negatively regulates GO:1900883 Also known as: down regulation of 17-methylnonadec-1-ene anabolism, down regulation of 17-methylnonadec-1-ene biosynthesis, down regulation of 17-methylnonadec-1-ene biosynthetic process, down regulation of 17-methylnonadec-1-ene formation, down regulation of 17-methylnonadec-1-ene synthesis, down-regulation of 17-methylnonadec-1-ene anabolism, down-regulation of 17-methylnonadec-1-ene biosynthesis, down-regulation of 17-methylnonadec-1-ene biosynthetic process, down-regulation of 17-methylnonadec-1-ene formation, down-regulation of 17-methylnonadec-1-ene synthesis, downregulation of 17-methylnonadec-1-ene anabolism, downregulation of 17-methylnonadec-1-ene biosynthesis, downregulation of 17-methylnonadec-1-ene biosynthetic process, downregulation of 17-methylnonadec-1-ene formation, downregulation of 17-methylnonadec-1-ene synthesis, inhibition of 17-methylnonadec-1-ene anabolism, inhibition of 17-methylnonadec-1-ene biosynthesis, inhibition of 17-methylnonadec-1-ene formation, inhibition of 17-methylnonadec-1-ene synthesis, negative regulation of 17-methylnonadec-1-ene anabolism, negative regulation of 17-methylnonadec-1-ene biosynthesis, negative regulation of 17-methylnonadec-1-ene formation, negative regulation of 17-methylnonadec-1-ene synthesis, inhibition of 17-methylnonadec-1-ene biosynthetic process